dehydrodolichyl diphosphate synthase complex [GO:1904423] (cellular component) Definition: A protein complex which is capable of dehydrodolichyl diphosphate synthase activity. References: PMID:25066056 Sources: GOC:TermGenie, GO_REF:0000088 Relationships: is a type of polyprenyl diphosphate synthase complex [GO:0032476]